{
  "gene_name": "Nipped-B-like protein",
  "term_label": "establishment of mitotic sister chromatid cohesion",
  "gene_symbol": "NIPBL",
  "gene": "UniProtKB:Q6KC79",
  "term_id": "GO:0034087"
}